protein-mitochondrial outer membrane tethering activity [GO:0180050] (molecular function) Sources: GOC:vw Relationships: is a type of protein-membrane adaptor activity [GO:0043495] Definition: The binding activity of a molecule that brings together a protein or protein complex and a mitochondrial outer membrane lipid or membrane-associated protein, in order to maintain the localization of the protein, or protein complex at a specific mitochondrial outer membrane location.